positive regulation of interleukin-19 production [GO:0032742] (biological process) Definition: Any process that activates or increases the frequency, rate, or extent of interleukin-19 production. Sources: GOC:mah Also known as: positive regulation of IL-19 production, up regulation of interleukin-19 production, up-regulation of interleukin-19 production, upregulation of interleukin-19 production, activation of interleukin-19 production, positive regulation of interleukin-19 biosynthetic process, stimulation of interleukin-19 production Relationships: is a type of positive regulation of cytokine production [GO:0001819]; is a type of regulation of interleukin-19 production [GO:0032662]; positively regulates interleukin-19 production [GO:0032622]